{
  "term_id": "GO:0007214",
  "gene_name": "Protein shisa-7",
  "gene_symbol": "SHISA7",
  "gene": "UniProtKB:A6NL88",
  "term_label": "gamma-aminobutyric acid signaling pathway"
}